{
  "term_id": "GO:0005634",
  "gene": "UniProtKB:Q9GZU2",
  "gene_symbol": "PEG3",
  "term_label": "nucleus",
  "gene_name": "Paternally-expressed gene 3 protein"
}